{
  "gene_symbol": "FAM83D",
  "term_label": "protein kinase binding",
  "term_id": "GO:0019901",
  "gene": "UniProtKB:Q9H4H8",
  "gene_name": "Protein FAM83D"
}